histone H3K79 dimethyltransferase activity [GO:0120506] (molecular function) Definition: Catalysis of the reaction: L-lysyl79-[histone H3] + 2 S-adenosyl-L-methionine = 2H+ + N6,N6-methyl-L-lysyl79-[histone H3] + 2 S-adenosyl-L-homocysteine. References: PMID:14732680, PMID:15371351 Relationships: is a type of histone H3K79 methyltransferase activity [GO:0031151] Note: Comment: Note that the residue position corresponds to the canonical human H3 histone (UniProtKB:P84243); this residue is conserved across all eukaryotes. Residue 1 is the first residue following removal of the initiating Methionine (Met). Note that each histone is encoded by multiple genes, and sequences may vary across different genes within an organism.